{
  "gene_symbol": "SIDT1",
  "gene": "UniProtKB:Q9NXL6",
  "gene_name": "SID1 transmembrane family member 1",
  "term_label": "RNA transmembrane transporter activity",
  "term_id": "GO:0051033"
}